{
  "term_id": "GO:0060294",
  "term_label": "cilium movement involved in cell motility",
  "gene_name": "Dynein axonemal heavy chain 8",
  "gene": "UniProtKB:Q96JB1",
  "gene_symbol": "DNAH8"
}